{
  "gene_name": "Class E basic helix-loop-helix protein 23",
  "gene_symbol": "BHLHE23",
  "term_label": "DNA-binding transcription factor activity, RNA polymerase II-specific",
  "gene": "UniProtKB:Q8NDY6",
  "term_id": "GO:0000981"
}